{
  "gene_name": "Signal recognition particle receptor subunit alpha",
  "term_id": "GO:0045047",
  "gene_symbol": "SRPRA",
  "term_label": "protein targeting to ER",
  "gene": "UniProtKB:P08240"
}